{
  "term_label": "organic acid metabolic process",
  "gene_symbol": "CYP2J2",
  "term_id": "GO:0006082",
  "gene": "UniProtKB:P51589",
  "gene_name": "Cytochrome P450 2J2"
}